{
  "term_label": "Unknown cellular component",
  "gene_symbol": "PRRT4",
  "gene": "UniProtKB:C9JH25",
  "gene_name": "Proline-rich transmembrane protein 4",
  "term_id": "UNKNOWN:0003"
}